{
  "term_label": "phosphatidylglycerophosphatase activity",
  "gene_symbol": "PTPMT1",
  "gene": "UniProtKB:Q8WUK0",
  "term_id": "GO:0008962",
  "gene_name": "Phosphatidylglycerophosphatase and protein-tyrosine phosphatase 1"
}